negative regulation of leukotriene production involved in inflammatory response [GO:0035492] (biological process) Sources: GOC:bf Definition: Any process that decreases the rate, frequency or extent of the synthesis or release of any leukotriene following a stimulus as part of an inflammatory response. Relationships: is a type of regulation of leukotriene production involved in inflammatory response [GO:0035490]; is_a negative regulation of inflammatory response [GO:0050728]; is a type of GO:0051241; negatively regulates leukotriene production involved in inflammatory response [GO:0002540]